{
  "term_label": "Unknown molecular function",
  "gene_symbol": "NYAP1",
  "term_id": "UNKNOWN:0001",
  "gene_name": "Neuronal tyrosine-phosphorylated phosphoinositide-3-kinase adapter 1",
  "gene": "UniProtKB:Q6ZVC0"
}